RNA polymerase II core promoter sequence-specific DNA binding [GO:0000979] (molecular function) Definition: Binding to a DNA sequence that is part of the core promoter of a RNA polymerase II-transcribed gene. Relationships: is a type of RNA polymerase II transcription regulatory region sequence-specific DNA binding [GO:0000977]; is a type of GO:0001046 References: PMID:12381658 Sources: GOC:pg, GOC:txnOH